picolinic acid biosynthetic process [GO:1905004] (biological process) References: PMID:19843166 Sources: GOC:PARL, GOC:TermGenie, GOC:bf, GO_REF:0000068 Relationships: is a type of GO:0072330; is a type of GO:0072525 Definition: The chemical reactions and pathways resulting in the formation of picolinic acid. Also known as: picolinate biosynthesis, picolinate biosynthetic process, picolinic acid anabolism, picolinic acid biosynthesis, picolinic acid formation, picolinic acid synthesis